{
  "gene_symbol": "SYT13",
  "gene": "UniProtKB:Q7L8C5",
  "term_id": "GO:0070382",
  "term_label": "exocytic vesicle",
  "gene_name": "Synaptotagmin-13"
}